regulation of chromosome attachment to the nuclear envelope [GO:0120264] (biological process) Relationships: is a type of GO:0010564; is a type of regulation of localization [GO:0032879]; regulates GO:0097240 Subtypes: GO:0120265, GO:0120266 Definition: Any process that modulates the frequency, rate, extent or location of chromosome attachment to the nuclear envelope. Sources: GOC:krc